B cell differentiation [GO:0030183] (biological process) Also known as: B lymphocyte differentiation, B-cell differentiation, B-lymphocyte differentiation, B cell development Definition: The process in which a precursor cell type acquires the specialized features of a B cell. A B cell is a lymphocyte of B lineage with the phenotype CD19-positive and capable of B cell mediated immunity. Subtypes: immature B cell differentiation [GO:0002327], GO:0002335 Relationships: is a type of lymphocyte differentiation [GO:0030098]; is a type of GO:0042113 Sources: GOC:mah, GO_REF:0000022 Regulation: regulated by regulation of B cell differentiation [GO:0045577]; RO_0002212 by GO:0045578; positively regulated by positive regulation of B cell differentiation [GO:0045579] Note: Note that immunologists typically use the word 'development' to refer to cells of B or T cell lineages undergoing the process that GO describes as 'cell differentiation'.